L-methionine biosynthetic process from homoserine via O-succinyl-L-homoserine and cystathionine [GO:0019281] (biological process) Sources: GOC:go_curators Also known as: L-methionine anabolism from homoserine via O-succinyl-L-homoserine and cystathionine, L-methionine formation from homoserine via O-succinyl-L-homoserine and cystathionine, L-methionine synthesis from homoserine via O-succinyl-L-homoserine and cystathionine, methionine biosynthetic process from homoserine via O-succinyl-L-homoserine and cystathionine Definition: The chemical reactions and pathways resulting in the formation of L-methionine from other compounds, including homoserine, via the intermediates O-succinyl-L-homoserine and cystathionine. Relationships: is a type of L-methionine biosynthetic process from L-homoserine via cystathionine [GO:0019279]